{
  "gene": "UniProtKB:Q8IZ07",
  "term_id": "GO:0005886",
  "gene_symbol": "ANKRD13A",
  "term_label": "plasma membrane",
  "gene_name": "Ankyrin repeat domain-containing protein 13A"
}